{
  "gene_name": "Uncharacterized protein DOCK8-AS1",
  "term_id": "UNKNOWN:0003",
  "gene": "UniProtKB:Q5T8R8",
  "gene_symbol": "DOCK8-AS1",
  "term_label": "Unknown cellular component"
}